{
  "gene_symbol": "RIDA",
  "gene": "UniProtKB:P52758",
  "gene_name": "2-iminobutanoate_2-iminopropanoate deaminase",
  "term_label": "deaminase activity",
  "term_id": "GO:0019239"
}